{
  "gene_symbol": "SLC35E1",
  "gene_name": "Solute carrier family 35 member E1",
  "term_id": "GO:0015297",
  "term_label": "antiporter activity",
  "gene": "UniProtKB:Q96K37"
}